positive regulation of cell communication by electrical coupling involved in cardiac conduction [GO:1901846] (biological process) Also known as: up regulation of cell communication by electrical coupling involved in cardiac conduction, up-regulation of cell communication by electrical coupling involved in cardiac conduction, upregulation of cell communication by electrical coupling involved in cardiac conduction, activation of cell communication by electrical coupling involved in cardiac conduction Relationships: is_a GO:0010650; is a type of regulation of cell communication by electrical coupling involved in cardiac conduction [GO:1901844]; RO_0002213 GO:0086064 Definition: Any process that activates or increases the frequency, rate or extent of cell communication by electrical coupling involved in cardiac conduction. References: PMID:17130302 Sources: GOC:BHF, GOC:TermGenie, GOC:rl